{
  "term_id": "UNKNOWN:0001",
  "gene_name": "Fibronectin type III domain-containing protein 4",
  "gene": "UniProtKB:Q9H6D8",
  "gene_symbol": "FNDC4",
  "term_label": "Unknown molecular function"
}